cupula development [GO:0048887] (biological process) Sources: ISBN:0125296509 Relationships: is a type of GO:0048856; is part of neuromast development [GO:0048884] Definition: The process whose specific outcome is the progression of the cupula over time, from its formation to the mature structure. The cupula is secreted by mantle cells and the ciliary bundles of all of the hair cells of the neuromast are embedded in it. The cupula provides a mechanical linkage between the hair cells and the external hydrodynamic environment. The cupula of superficial neuromasts grows continuously, while the height of the cupula of canal neuromasts is limited by canal diameter. Subtypes: anterior lateral line neuromast cupula development [GO:0048904], posterior lateral line neuromast cupula development [GO:0048921]